{
  "gene": "UniProtKB:P17676",
  "gene_name": "CCAAT_enhancer-binding protein beta",
  "term_label": "RNA polymerase II cis-regulatory region sequence-specific DNA binding",
  "gene_symbol": "CEBPB",
  "term_id": "GO:0000978"
}